epithelium development [GO:0060429] (BP) Relationships: is a type of tissue development [GO:0009888] Definition: The process whose specific outcome is the progression of an epithelium over time, from its formation to the mature structure. An epithelium is a tissue that covers the internal or external surfaces of an anatomical structure. Subtypes: GO:0001840, GO:0003158, GO:0003313, GO:0003406, neural tube development [GO:0021915], embryonic heart tube development [GO:0035050], GO:0035846, pericardium development [GO:0060039], lung epithelium development [GO:0060428], somite development [GO:0061053], urethra epithelium development [GO:0061071], seminal vesicle epithelium development [GO:0061108], mammary gland epithelium development [GO:0061180], renal tubule development [GO:0061326], GO:0071599, kidney epithelium development [GO:0072073], ureter urothelium development [GO:0072190], skin epidermis development [GO:0098773], epithelium regeneration [GO:1990399] Sources: GOC:dph, GOC:mtg_lung